{
  "term_id": "GO:0030218",
  "term_label": "erythrocyte differentiation",
  "gene_name": "Heme transporter FLVCR1",
  "gene_symbol": "FLVCR1",
  "gene": "UniProtKB:Q9Y5Y0"
}